{
  "term_id": "GO:0061630",
  "gene_symbol": "RNF4",
  "gene_name": "E3 ubiquitin-protein ligase RNF4",
  "term_label": "ubiquitin protein ligase activity",
  "gene": "UniProtKB:P78317"
}